detection of low humidity [GO:0098517] (biological process) Definition: The series of events in which low humidity is detected and converted into a molecular signal. Sources: GOC:dos Relationships: is a type of detection of humidity [GO:0098513] Subtypes: detection of low humidity stimulus involved in sensory perception [GO:0098515]